{
  "term_id": "GO:0042632",
  "term_label": "cholesterol homeostasis",
  "gene_name": "ATP-binding cassette sub-family G member 5",
  "gene_symbol": "ABCG5",
  "gene": "UniProtKB:Q9H222"
}